{
  "term_label": "SMAD protein signal transduction",
  "gene_symbol": "SMAD2",
  "gene": "UniProtKB:Q15796",
  "term_id": "GO:0060395",
  "gene_name": "Mothers against decapentaplegic homolog 2"
}